{
  "gene_symbol": "RNF186",
  "gene_name": "E3 ubiquitin-protein ligase RNF186",
  "term_label": "protein autoubiquitination",
  "term_id": "GO:0051865",
  "gene": "UniProtKB:Q9NXI6"
}